{
  "term_id": "GO:0006487",
  "term_label": "protein N-linked glycosylation",
  "gene_symbol": "FUT8",
  "gene": "UniProtKB:Q9BYC5",
  "gene_name": "Alpha-(1,6)-fucosyltransferase"
}